{
  "term_id": "UNKNOWN:0001",
  "term_label": "Unknown molecular function",
  "gene": "UniProtKB:O43820",
  "gene_symbol": "HYAL3",
  "gene_name": "Hyaluronidase-3"
}